O antigen polymerase activity [GO:0008755] (molecular function) Relationships: is a type of hexosyltransferase activity [GO:0016758] Also known as: O-antigen polymerase activity References: PMID:12045108 Sources: GOC:jl Definition: Catalysis of the polymerization of o-antigen chains. O-antigens are tetra- and pentasaccharide repeat units of the cell walls of Gram-negative bacteria and are a component of lipopolysaccharide.